{
  "term_id": "GO:0006887",
  "gene": "UniProtKB:Q8WXH6",
  "gene_name": "Ras-related protein Rab-40A",
  "term_label": "exocytosis",
  "gene_symbol": "RAB40A"
}